cytoplasmic stress granule [GO:0010494] (cellular component) Relationships: is a type of cytoplasmic ribonucleoprotein granule [GO:0036464] Definition: A dense aggregation in the cytosol composed of proteins and RNAs that appear when the cell is under stress. References: PMID:17284590, PMID:17601829, PMID:17967451, PMID:20368989 Sources: GOC:ans Also known as: cytoplasmic mRNP granule, stress granule